{
  "gene_symbol": "MDFIC2",
  "gene": "UniProtKB:A0A1B0GVS7",
  "term_label": "negative regulation of DNA-templated transcription",
  "term_id": "GO:0045892",
  "gene_name": "MyoD family inhibitor domain-containing protein 2"
}